{
  "term_label": "mitochondrial matrix",
  "gene_symbol": "LYRM7",
  "gene": "UniProtKB:Q5U5X0",
  "term_id": "GO:0005759",
  "gene_name": "Complex III assembly factor LYRM7"
}